{
  "term_label": "Unknown molecular function",
  "gene_name": "N-terminal EF-hand calcium-binding protein 2",
  "gene_symbol": "NECAB2",
  "term_id": "UNKNOWN:0001",
  "gene": "UniProtKB:Q7Z6G3"
}